{
  "gene": "UniProtKB:P49682",
  "gene_symbol": "CXCR3",
  "term_label": "C-C chemokine receptor activity",
  "gene_name": "C-X-C chemokine receptor type 3",
  "term_id": "GO:0016493"
}